MutSgamma complex [GO:0062128] (cellular component) References: PMID:27648641, PMID:7622037, PMID:8001134, PMID:9374523 Relationships: is a type of mismatch repair complex [GO:0032300]; is a type of GO:0140513 Definition: A heterodimer involved in the stabilization of DNA recombination intermediates, the promotion of crossover recombination, and the proper assembly of the synaptonemal complex in meiotic prophase nuclei. In yeast the complex consists of two subunits, Msh4 and Msh5. Also known as: Msh4-Msh5 complex